maintenance of oocyte nucleus location involved in oocyte dorsal/ventral axis specification [GO:0042070] (biological process) Sources: GOC:dph, GOC:mah, GOC:mtg_sensu, GOC:tb Also known as: maintenance of oocyte nucleus localization during oocyte axis determination, maintenance of oocyte nucleus position during oocyte axis determination, oocyte axis determination, maintenance of oocyte nucleus localization, oocyte axis determination, maintenance of oocyte nucleus position, oocyte axis determination, oocyte nucleus anchoring, oocyte nucleus anchoring during oocyte axis determination, maintenance of oocyte nucleus location involved in oocyte dorsal-ventral axis specification, maintenance of oocyte nucleus location involved in oocyte dorsal/ventral axis determination, maintenance of oocyte nucleus location involved in oocyte dorsoventral axis specification Relationships: is a type of maintenance of nucleus location [GO:0051658]; is a type of GO:0051663 Definition: Maintenance of the oocyte nucleus in a particular position within the cell during the establishment and maintenance of the axes of the oocyte. An example of this process is found In Drosophila melanogaster.